response to strigolactone [GO:1902347] (biological process) Also known as: response to strigolactone analog GR24 Relationships: is a type of GO:0033993; is a type of response to oxygen-containing compound [GO:1901700] References: PMID:23893171 Sources: GOC:TermGenie Subtypes: cellular response to strigolactone [GO:1902348] Definition: Any process that results in a change in state or activity of a cell or an organism (in terms of movement, secretion, enzyme production, gene expression, etc.) as a result of a strigolactone stimulus.